{
  "term_label": "regulation of meiosis I",
  "gene_name": "Wee1-like protein kinase 2",
  "gene_symbol": "WEE2",
  "term_id": "GO:0060631",
  "gene": "UniProtKB:P0C1S8"
}